{
  "term_label": "cytokine-mediated signaling pathway",
  "term_id": "GO:0019221",
  "gene_name": "Non-receptor tyrosine-protein kinase TYK2",
  "gene_symbol": "TYK2",
  "gene": "UniProtKB:P29597"
}